{
  "gene_symbol": "SRMS",
  "term_label": "plasma membrane",
  "term_id": "GO:0005886",
  "gene_name": "Tyrosine-protein kinase Srms",
  "gene": "UniProtKB:Q9H3Y6"
}